{
  "gene": "UniProtKB:Q8WXF1",
  "term_id": "GO:0006355",
  "term_label": "regulation of DNA-templated transcription",
  "gene_symbol": "PSPC1",
  "gene_name": "Paraspeckle component 1"
}